{
  "term_label": "Unknown molecular function",
  "gene": "UniProtKB:Q8TCB0",
  "term_id": "UNKNOWN:0001",
  "gene_name": "Interferon-induced protein 44",
  "gene_symbol": "IFI44"
}